{
  "term_label": "Unknown cellular component",
  "gene": "UniProtKB:Q6T423",
  "term_id": "UNKNOWN:0003",
  "gene_symbol": "SLC22A25",
  "gene_name": "Solute carrier family 22 member 25"
}